all-trans-neoxanthin catabolic process [GO:1901832] (biological process) References: PMID:11029576 Sources: GOC:TermGenie, GOC:yaf, MetaCyc:PWY-6809, UniPathway:UPA00388 Also known as: all-trans-neoxanthin breakdown, all-trans-neoxanthin catabolism, all-trans-neoxanthin degradation, neoxanthin breakdown, neoxanthin catabolic process, neoxanthin catabolism, neoxanthin degradation Relationships: is a type of xanthophyll catabolic process [GO:0016124]; is a type of epoxide metabolic process [GO:0097176]; is a type of olefinic compound catabolic process [GO:0120256]; is a type of ether catabolic process [GO:1901502] Definition: The chemical reactions and pathways resulting in the breakdown of all-trans-neoxanthin.